phenanthrene catabolic process via trans-9(R),10(R)-dihydrodiolphenanthrene [GO:0018956] (biological process) Sources: UM-BBD_pathwayID:pha3 Definition: The chemical reactions and pathways resulting in the breakdown of phenanthrene, a tricyclic aromatic hydrocarbon, where trans-9(R),10(R)-dihydrodiolphenanthrene is the principal intermediate metabolite. Also known as: phenanthrene breakdown via trans-9(R),10(R)-dihydrodiolphenanthrene, phenanthrene degradation via trans-9(R),10(R)-dihydrodiolphenanthrene Relationships: is a type of phenanthrene catabolic process [GO:0042216]